{
  "gene_symbol": "MBTD1",
  "gene": "UniProtKB:Q05BQ5",
  "term_id": "GO:0042393",
  "term_label": "histone binding",
  "gene_name": "MBT domain-containing protein 1"
}